{
  "term_id": "GO:0000981",
  "term_label": "DNA-binding transcription factor activity, RNA polymerase II-specific",
  "gene_symbol": "ZNF442",
  "gene": "UniProtKB:Q9H7R0",
  "gene_name": "Zinc finger protein 442"
}